{
  "term_label": "positive regulation of myoblast differentiation",
  "gene_name": "Myoblast determination protein 1",
  "gene_symbol": "MYOD1",
  "term_id": "GO:0045663",
  "gene": "UniProtKB:P15172"
}